neuropeptide secretion from presynapse [GO:0099539] (biological process) Relationships: is a type of peptide secretion [GO:0002790]; is a type of presynaptic dense core vesicle exocytosis [GO:0099525]; is part of GO:0099538 Also known as: neuropeptide secretion from presynapse via dense core granule exocytosis References: PMID:17553987, PMID:24653208 Definition: The secretion of neuropeptides contained within a dense core vesicle by fusion of the granule with the presynaptic membrane, stimulated by a rise in cytosolic calcium ion concentration.